{
  "term_id": "GO:0005743",
  "gene": "UniProtKB:P12235",
  "gene_symbol": "SLC25A4",
  "gene_name": "ADP_ATP translocase 1",
  "term_label": "mitochondrial inner membrane"
}